{
  "gene_symbol": "MYL9",
  "term_id": "GO:0016460",
  "gene_name": "Myosin regulatory light polypeptide 9",
  "term_label": "myosin II complex",
  "gene": "UniProtKB:P24844"
}